{
  "term_label": "Unknown biological process",
  "gene_name": "Putative uncharacterized protein FLJ26174",
  "gene": "UniProtKB:Q6ZPA2",
  "term_id": "UNKNOWN:0002",
  "gene_symbol": "Q6ZPA2"
}